{
  "gene": "UniProtKB:Q1AE95",
  "term_id": "UNKNOWN:0002",
  "gene_symbol": "TMEM183BP",
  "term_label": "Unknown biological process",
  "gene_name": "Putative transmembrane protein 183BP"
}